{
  "gene": "UniProtKB:P18077",
  "term_label": "cytoplasmic translation",
  "gene_name": "Large ribosomal subunit protein eL33",
  "term_id": "GO:0002181",
  "gene_symbol": "RPL35A"
}